{
  "term_label": "intracellular protein transport",
  "gene_name": "Putative ADP-ribosylation factor-like protein 5C",
  "term_id": "GO:0006886",
  "gene_symbol": "ARL5C",
  "gene": "UniProtKB:A6NH57"
}